{
  "term_label": "Unknown molecular function",
  "gene_symbol": "TMEM244",
  "gene_name": "Transmembrane protein 244",
  "term_id": "UNKNOWN:0001",
  "gene": "UniProtKB:Q5VVB8"
}